structural constituent of postsynaptic intermediate filament cytoskeleton [GO:0099184] (molecular function) Sources: GOC:dos Relationships: is a type of structural constituent of cytoskeleton [GO:0005200]; is a type of structural constituent of postsynapse [GO:0099186]; is part of postsynaptic intermediate filament cytoskeleton organization [GO:0099185]; occurs in postsynaptic intermediate filament cytoskeleton [GO:0099160] Definition: The action of a molecule that contributes to the structural integrity of a postsynaptic intermediate filament cytoskeleton.